{
  "term_label": "lipid catabolic process",
  "term_id": "GO:0016042",
  "gene": "UniProtKB:Q53H76",
  "gene_symbol": "PLA1A",
  "gene_name": "Phospholipase A1 member A"
}